{
  "term_label": "FATZ binding",
  "term_id": "GO:0051373",
  "gene": "UniProtKB:Q9NPC6",
  "gene_symbol": "MYOZ2",
  "gene_name": "Myozenin-2"
}